regulation of neutrophil mediated cytotoxicity [GO:0070948] (biological process) Subtypes: regulation of neutrophil mediated killing of symbiont cell [GO:0070949], negative regulation of neutrophil mediated cytotoxicity [GO:0070954], positive regulation of neutrophil mediated cytotoxicity [GO:0070960] Definition: Any process that modulates the rate, frequency or extent of neutrophil mediated killing of a target cell, the directed killing of a target cell by a neutrophil. Also known as: regulation of neutrophil mediated cell killing Sources: GOC:add, GOC:mah Relationships: is a type of regulation of leukocyte mediated cytotoxicity [GO:0001910]; is a type of regulation of myeloid leukocyte mediated immunity [GO:0002886]; regulates neutrophil mediated cytotoxicity [GO:0070942]